{
  "gene_name": "Transmembrane and coiled-coil domains protein 2",
  "term_label": "Unknown molecular function",
  "gene": "UniProtKB:O75069",
  "term_id": "UNKNOWN:0001",
  "gene_symbol": "TMCC2"
}